protein-glycine ligase activity, initiating [GO:0070736] (MF) Definition: Catalysis of the posttranslational transfer of a glycine residue to the gamma-carboxyl group(s) of one or more specific glutamate residues on a target protein. References: PMID:19524510 Sources: GOC:mah Relationships: is a type of protein-glycine ligase activity [GO:0070735] Also known as: protein glycylase activity, initiating